mesenchymal smoothened signaling pathway involved in prostate gland development [GO:0060783] (biological process) References: PMID:12221011 Relationships: is a type of GO:0007224; is part of epithelial-mesenchymal signaling involved in prostate gland development [GO:0060738] Definition: The series of molecular signals generated as a consequence of activation of the transmembrane Smoothened-type protein in the mesenchymal cells of the prostate that contribute to the progression of the prostate over time. This process contributes to lung development. Also known as: mesenchymal hedgehog signaling pathway involved in prostate gland development, mesenchymal hh signaling pathway involved in prostate gland development, mesenchymal smoothened signalling pathway involved in prostate gland development